{
  "gene_symbol": "SLC5A12",
  "term_label": "sodium ion transport",
  "gene": "UniProtKB:Q1EHB4",
  "term_id": "GO:0006814",
  "gene_name": "Sodium-coupled monocarboxylate transporter 2"
}